{
  "gene_name": "Zinc finger and SCAN domain-containing protein 16",
  "gene": "UniProtKB:Q9H4T2",
  "term_label": "DNA-binding transcription factor activity, RNA polymerase II-specific",
  "gene_symbol": "ZSCAN16",
  "term_id": "GO:0000981"
}